cellular response to chemical stress [GO:0062197] (BP) References: PMID:26653712 Subtypes: cellular response to oxidative stress [GO:0034599], GO:0036447, GO:0071455, cellular response to hydrostatic pressure [GO:0071464], GO:0071470, cellular response to nitrosative stress [GO:0071500], cellular response to boron-containing substance deprivation [GO:0080169], cellular stress response to acidic pH [GO:1990451], response to manganese-induced endoplasmic reticulum stress [GO:1990737] Relationships: is a type of GO:0033554; is a type of cellular response to chemical stimulus [GO:0070887] Definition: Any process that results in a change in state or activity of a cell (in terms of movement, secretion, enzyme production, gene expression, etc.) as a result of a chemical stimulus indicating the organism is under stress.